positive regulation of t-SNARE clustering [GO:1904034] (biological process) References: PMID:22528485 Sources: GOC:TermGenie, GO_REF:0000058 Also known as: up regulation of t-SNARE clustering, up-regulation of t-SNARE clustering, upregulation of t-SNARE clustering, activation of t-SNARE clustering Relationships: is a type of regulation of t-SNARE clustering [GO:1904032]; is a type of positive regulation of protein localization to membrane [GO:1905477]; positively regulates GO:1990656 Definition: Any process that activates or increases the frequency, rate or extent of t-SNARE clustering.